negative regulation of protein K63-linked deubiquitination [GO:1903005] (BP) Definition: Any process that stops, prevents or reduces the frequency, rate or extent of protein K63-linked deubiquitination. Relationships: is_a negative regulation of protein deubiquitination [GO:0090086]; is a type of GO:1903004; RO_0002212 GO:0070536 References: PMID:22970133 Sources: GOC:PARL, GOC:TermGenie, GOC:bf, GO_REF:0000058 Also known as: down regulation of protein K63-linked deubiquitination, down-regulation of protein K63-linked deubiquitination, downregulation of protein K63-linked deubiquitination, inhibition of protein K63-linked deubiquitination